{
  "gene": "UniProtKB:Q9Y6Y0",
  "gene_name": "Influenza virus NS1A-binding protein",
  "gene_symbol": "IVNS1ABP",
  "term_label": "proteasome-mediated ubiquitin-dependent protein catabolic process",
  "term_id": "GO:0043161"
}